{
  "gene_name": "Sodium_potassium-transporting ATPase subunit beta-2",
  "gene_symbol": "ATP1B2",
  "term_id": "GO:0001671",
  "term_label": "ATPase activator activity",
  "gene": "UniProtKB:P14415"
}